positive regulation of extrinsic apoptotic signaling pathway via death domain receptors [GO:1902043] (biological process) Subtypes: positive regulation of TRAIL-activated apoptotic signaling pathway [GO:1903984] Definition: Any process that activates or increases the frequency, rate or extent of extrinsic apoptotic signaling pathway via death domain receptors. Also known as: up regulation of extrinsic apoptotic signaling pathway via death domain receptors, up-regulation of extrinsic apoptotic signaling pathway via death domain receptors, upregulation of extrinsic apoptotic signaling pathway via death domain receptors, activation of death receptor-mediated apoptosis, activation of extrinsic apoptotic signaling pathway via death domain receptors, positive regulation of death receptor-mediated apoptosis, up regulation of death receptor-mediated apoptosis, up-regulation of death receptor-mediated apoptosis, upregulation of death receptor-mediated apoptosis Relationships: is a type of regulation of extrinsic apoptotic signaling pathway via death domain receptors [GO:1902041]; is a type of GO:2001238; positively regulates GO:0008625 References: PMID:17245429 Sources: GOC:TermGenie